{
  "term_id": "GO:0032545",
  "gene_symbol": "RRP7A",
  "gene": "UniProtKB:Q9Y3A4",
  "gene_name": "Ribosomal RNA-processing protein 7 homolog A",
  "term_label": "CURI complex"
}